{
  "gene": "UniProtKB:Q9HAR2",
  "gene_symbol": "ADGRL3",
  "term_label": "axon",
  "term_id": "GO:0030424",
  "gene_name": "Adhesion G protein-coupled receptor L3"
}